{
  "gene_symbol": "FAM131B",
  "term_id": "UNKNOWN:0003",
  "term_label": "Unknown cellular component",
  "gene_name": "Protein FAM131B",
  "gene": "UniProtKB:Q86XD5"
}